{
  "gene": "UniProtKB:Q8N5M9",
  "gene_name": "Protein jagunal homolog 1",
  "gene_symbol": "JAGN1",
  "term_id": "GO:0007029",
  "term_label": "endoplasmic reticulum organization"
}